{
  "gene_name": "Receptor-type tyrosine-protein phosphatase F",
  "gene_symbol": "PTPRF",
  "gene": "UniProtKB:P10586",
  "term_label": "nervous system development",
  "term_id": "GO:0007399"
}